oxidation-dependent protein catabolic process [GO:0070407] (biological process) Relationships: is a type of modification-dependent protein catabolic process [GO:0019941] Also known as: oxidation-dependent protein breakdown, oxidation-dependent protein catabolism, oxidation-dependent protein degradation, oxidation-dependent proteolysis, oxidized protein catabolic process Definition: The chemical reactions and pathways resulting in the breakdown of a protein or peptide by hydrolysis of its peptide bonds, initiated by the oxidation of one or more amino acid residues in the protein. Sources: GOC:mah